{
  "term_label": "Unknown cellular component",
  "gene": "UniProtKB:A0A0U1RQF7",
  "term_id": "UNKNOWN:0003",
  "gene_symbol": "DPEP2NB",
  "gene_name": "DPEP2 neighbor protein"
}